{
  "gene_symbol": "NHP2",
  "term_label": "snRNA pseudouridine synthesis",
  "term_id": "GO:0031120",
  "gene_name": "H_ACA ribonucleoprotein complex subunit 2",
  "gene": "UniProtKB:Q9NX24"
}